endoplasmic reticulum chaperone complex [GO:0034663] (CC) Relationships: is a type of endoplasmic reticulum protein-containing complex [GO:0140534] Definition: A protein complex that is located in the endoplasmic reticulum and is composed of chaperone proteins, including BiP, GRP94; CaBP1, protein disulfide isomerase (PDI), ERdj3, cyclophilin B, ERp72, GRP170, UDP-glucosyltransferase, and SDF2-L1. References: PMID:12475965 Also known as: ER chaperone complex, ER network complex, endoplasmic reticulum network complex